{
  "term_id": "GO:0007631",
  "gene": "UniProtKB:P01303",
  "gene_symbol": "NPY",
  "gene_name": "Pro-neuropeptide Y",
  "term_label": "feeding behavior"
}